{
  "gene_symbol": "KLK13",
  "gene": "UniProtKB:Q9UKR3",
  "term_label": "secretory granule",
  "gene_name": "Kallikrein-13",
  "term_id": "GO:0030141"
}